{
  "gene": "UniProtKB:Q08AN1",
  "gene_name": "Zinc finger protein 616",
  "term_id": "GO:0000978",
  "gene_symbol": "ZNF616",
  "term_label": "RNA polymerase II cis-regulatory region sequence-specific DNA binding"
}